atrazine catabolic process to urea [GO:0019623] (biological process) Also known as: atrazine breakdown to urea, atrazine degradation to urea Relationships: is a type of atrazine catabolic process [GO:0019381]; is a type of urea metabolic process [GO:0019627]; is a type of amide catabolic process [GO:0043605] Sources: GOC:jl Definition: The chemical reactions and pathways resulting in the breakdown of atrazine, a triazine ring-containing herbicide, into urea.